{
  "gene": "UniProtKB:Q9BXU0",
  "gene_symbol": "TEX12",
  "term_id": "GO:0000801",
  "gene_name": "Testis-expressed protein 12",
  "term_label": "central element"
}